{
  "gene_name": "Protocadherin beta-7",
  "gene_symbol": "PCDHB7",
  "term_id": "GO:0050839",
  "term_label": "cell adhesion molecule binding",
  "gene": "UniProtKB:Q9Y5E2"
}